{
  "gene_symbol": "SFTPB",
  "gene_name": "Pulmonary surfactant-associated protein B",
  "gene": "UniProtKB:P07988",
  "term_id": "UNKNOWN:0002",
  "term_label": "Unknown biological process"
}